{
  "gene_name": "T cell receptor alpha variable 7",
  "term_label": "Unknown molecular function",
  "term_id": "UNKNOWN:0001",
  "gene_symbol": "TRAV7",
  "gene": "UniProtKB:A0A075B6U4"
}